{
  "gene_symbol": "ZNF821",
  "term_id": "GO:0000978",
  "gene": "UniProtKB:O75541",
  "term_label": "RNA polymerase II cis-regulatory region sequence-specific DNA binding",
  "gene_name": "Zinc finger protein 821"
}